{
  "term_label": "cytoplasmic translational initiation",
  "term_id": "GO:0002183",
  "gene_symbol": "EIF2B3",
  "gene_name": "Translation initiation factor eIF-2B subunit gamma",
  "gene": "UniProtKB:Q9NR50"
}